protein insertion into membrane raft [GO:0071210] (biological process) Relationships: is a type of protein insertion into membrane [GO:0051205]; is part of membrane raft organization [GO:0031579] Subtypes: protein insertion into plasma membrane raft [GO:0044859] Also known as: establishment of protein localization to membrane raft Definition: The process in which a protein is incorporated into a membrane raft. Membrane rafts are small (10-200 nm), heterogeneous, highly dynamic, sterol- and sphingolipid-enriched membrane domains that compartmentalize cellular processes. Sources: GOC:mah